{
  "term_id": "GO:0005813",
  "gene_name": "Speriolin",
  "term_label": "centrosome",
  "gene": "UniProtKB:Q76KD6",
  "gene_symbol": "SPATC1"
}